negative regulation of extrinsic apoptotic signaling pathway in absence of ligand [GO:2001240] (biological process) Definition: Any process that stops, prevents or reduces the frequency, rate or extent of extrinsic apoptotic signaling pathway in absence of ligand. Sources: GOC:mtg_apoptosis Also known as: negative regulation of extrinsic apoptotic signalling pathway in absence of ligand, negative regulation of extrinsic apoptosis in absence of ligand, negative regulation of dependence receptor signaling pathway Relationships: is a type of negative regulation of signal transduction in absence of ligand [GO:1901099]; is a type of negative regulation of extrinsic apoptotic signaling pathway [GO:2001237]; is a type of regulation of extrinsic apoptotic signaling pathway in absence of ligand [GO:2001239]; negatively regulates GO:0097192